ABC-type nickel transporter activity [GO:0015413] (molecular function) Definition: Enables the transfer of a solute or solutes from one side of a membrane to the other according to the reaction: ATP + H2O + Ni2+(out) = ADP + phosphate + Ni2+(in). Relationships: is a type of GO:0015099; is a type of ATPase-coupled monoatomic cation transmembrane transporter activity [GO:0019829]; is a type of GO:0140359 Sources: RHEA:15557 Also known as: nickel ABC transporter, nickel ABC transporter activity, ATP-dependent nickel transmembrane transporter activity, ATPase-coupled nickel transmembrane transporter activity, nickel porter activity, nickel transporting ATPase activity, nickel-transporting ATPase activity